{
  "term_label": "positive regulation of cell migration",
  "gene_name": "C-X-C motif chemokine 16",
  "term_id": "GO:0030335",
  "gene": "UniProtKB:Q9H2A7",
  "gene_symbol": "CXCL16"
}